{
  "gene": "UniProtKB:Q9BQE6",
  "gene_symbol": "LBHD1",
  "term_label": "positive regulation of DNA-templated transcription",
  "term_id": "GO:0045893",
  "gene_name": "LBH domain-containing protein 1"
}